{
  "gene": "UniProtKB:C9J069",
  "gene_name": "Apical junction component 1 homolog",
  "gene_symbol": "AJM1",
  "term_id": "GO:0043296",
  "term_label": "apical junction complex"
}